{
  "gene_symbol": "RGS19",
  "term_id": "GO:0005096",
  "gene_name": "Regulator of G-protein signaling 19",
  "term_label": "GTPase activator activity",
  "gene": "UniProtKB:P49795"
}